DNA transport [GO:0051027] (biological process) Subtypes: DNA import into cell involved in transformation [GO:0009290] Definition: The directed movement of RNA, deoxyribonucleic acid, into, out of or within a cell, or between cells, by means of some agent such as a transporter or pore. Relationships: is a type of GO:0050657 Sources: GOC:ai